{
  "gene_name": "Homeobox protein Nkx-2.5",
  "term_id": "GO:0030154",
  "term_label": "cell differentiation",
  "gene_symbol": "NKX2-5",
  "gene": "UniProtKB:P52952"
}